locus ceruleus maturation [GO:0021706] (biological process) Definition: A developmental process, independent of morphogenetic (shape) change, that is required for the locus ceruleus to attain its fully functional state. The locus ceruleus is a dense cluster of neurons within the dorsorostral pons. This nucleus is the major location of neurons that release norepinephrine throughout the brain, and is responsible for physiological responses to stress and panic. Relationships: is a type of GO:0071695; is part of pons maturation [GO:0021586]; is part of locus ceruleus development [GO:0021703] Sources: GOC:cls, GOC:dgh, GOC:dph, GOC:jid, GO_REF:0000021